{
  "gene": "UniProtKB:Q9H2X6",
  "term_label": "intrinsic apoptotic signaling pathway in response to DNA damage by p53 class mediator",
  "gene_name": "Homeodomain-interacting protein kinase 2",
  "term_id": "GO:0042771",
  "gene_symbol": "HIPK2"
}